{
  "gene_symbol": "LHX3",
  "gene": "UniProtKB:Q9UBR4",
  "term_id": "GO:0005634",
  "term_label": "nucleus",
  "gene_name": "LIM_homeobox protein Lhx3"
}